{
  "term_id": "GO:0005737",
  "term_label": "cytoplasm",
  "gene": "UniProtKB:Q07960",
  "gene_symbol": "ARHGAP1",
  "gene_name": "Rho GTPase-activating protein 1"
}